{
  "gene_name": "Kelch repeat and BTB domain-containing protein 3",
  "gene": "UniProtKB:Q8NAB2",
  "term_label": "cytoplasm",
  "gene_symbol": "KBTBD3",
  "term_id": "GO:0005737"
}